{
  "gene_name": "Ubiquitin carboxyl-terminal hydrolase 11",
  "gene_symbol": "USP11",
  "term_id": "UNKNOWN:0001",
  "gene": "UniProtKB:P51784",
  "term_label": "Unknown molecular function"
}